{
  "term_label": "detection of calcium ion",
  "gene_name": "Calmodulin-like protein 3",
  "term_id": "GO:0005513",
  "gene": "UniProtKB:P27482",
  "gene_symbol": "CALML3"
}